{
  "gene_symbol": "H2AX",
  "gene_name": "Histone H2AX",
  "term_label": "nucleus",
  "term_id": "GO:0005634",
  "gene": "UniProtKB:P16104"
}